{
  "term_id": "UNKNOWN:0001",
  "gene": "UniProtKB:Q9BQT8",
  "term_label": "Unknown molecular function",
  "gene_symbol": "SLC25A21",
  "gene_name": "Mitochondrial 2-oxodicarboxylate carrier"
}